clathrin-sculpted gamma-aminobutyric acid transport vesicle [GO:0061200] (cellular component) Sources: GOC:dph Also known as: clathrin sculpted GABA transport vesicle, clathrin sculpted gamma-aminobutyric acid transport vesicle Relationships: is a type of clathrin-sculpted vesicle [GO:0060198] Definition: A clathrin-sculpted lipid bilayer membrane-enclosed vesicle after clathrin release and containing gamma-aminobutyric acid transport vesicle.